{
  "term_label": "RNA nuclease activity",
  "gene": "UniProtKB:Q93091",
  "gene_name": "Ribonuclease K6",
  "term_id": "GO:0004540",
  "gene_symbol": "RNASE6"
}